austinol catabolic process [GO:1900559] (biological process) Sources: GOC:TermGenie, GOC:di Definition: The chemical reactions and pathways resulting in the breakdown of austinol. Also known as: austinol breakdown, austinol catabolism, austinol degradation Relationships: is a type of catabolic process [GO:0009056]